{
  "gene": "UniProtKB:P25815",
  "term_label": "cytoplasm",
  "gene_symbol": "S100P",
  "gene_name": "Protein S100-P",
  "term_id": "GO:0005737"
}